{
  "gene": "UniProtKB:Q96HH6",
  "term_id": "UNKNOWN:0002",
  "term_label": "Unknown biological process",
  "gene_symbol": "TMEM19",
  "gene_name": "Transmembrane protein 19"
}